{
  "term_label": "antigen binding",
  "term_id": "GO:0003823",
  "gene_name": "Immunoglobulin heavy variable 3-74",
  "gene_symbol": "IGHV3-74",
  "gene": "UniProtKB:A0A0B4J1X5"
}